sequestering of calcium ion [GO:0051208] (BP) Sources: GOC:ai Definition: The process of binding or confining calcium ions such that they are separated from other components of a biological system. Also known as: calcium ion (Ca2+) retention, calcium ion (Ca2+) sequestering, calcium ion (Ca2+) sequestration, calcium ion (Ca2+) storage, retention of calcium ion (Ca2+), sequestering of calcium ion (Ca2+), sequestration of calcium ion (Ca2+), storage of calcium ion (Ca2+), calcium ion storage activity, negative regulation of calcium ion (Ca2+) transport Regulation: regulated by regulation of sequestering of calcium ion [GO:0051282]; negatively regulated by negative regulation of sequestering of calcium ion [GO:0051283]; positively regulated by GO:0051284 Relationships: is_a GO:0051651; is part of intracellular calcium ion homeostasis [GO:0006874]